{
  "gene": "UniProtKB:Q9UNG2",
  "gene_name": "Tumor necrosis factor ligand superfamily member 18",
  "term_label": "tumor necrosis factor-mediated signaling pathway",
  "term_id": "GO:0033209",
  "gene_symbol": "TNFSF18"
}